regulation of basophil differentiation [GO:0045640] (biological process) Definition: Any process that modulates the frequency, rate or extent of basophil differentiation. Relationships: is a type of regulation of granulocyte differentiation [GO:0030852]; regulates GO:0030221 Sources: GOC:go_curators Subtypes: negative regulation of basophil differentiation [GO:0045641], positive regulation of basophil differentiation [GO:0045642]